cellular response to stimulus [GO:0051716] (biological process) Subtypes: establishment of competence for transformation [GO:0030420], GO:0031669, cellular response to stress [GO:0033554], cellular pigment accumulation [GO:0043482], skeletal muscle fiber adaptation [GO:0043503], GO:0061646, GO:0061862, cellular response to chemical stimulus [GO:0070887], cellular response to biotic stimulus [GO:0071216], GO:0071402, cellular response to cell-matrix adhesion [GO:0071460], cellular response to environmental stimulus [GO:0104004], cellular response to cell wall damage [GO:1990394] Sources: GOC:bf, GOC:jl Relationships: is a type of cellular process [GO:0009987]; is a type of response to stimulus [GO:0050896] Definition: Any process that results in a change in state or activity of a cell (in terms of movement, secretion, enzyme production, gene expression, etc.) as a result of a stimulus. The process begins with detection of the stimulus by a cell and ends with a change in state or activity or the cell. Note: Note that this term is in the subset of terms that should not be used for direct gene product annotation. Instead, select a child term or, if no appropriate child term exists, please request a new term. Direct annotations to this term may be amended during annotation QC.